brainstem precerebellar neuron precursor migration [GO:0021949] (biological process) References: PMID:15157725 Sources: GOC:cls, GOC:dgh, GOC:dph, GOC:jid, GO_REF:0000021 Definition: The early migration of a precerebellar neuronal precursor in which a cell move from the rhombic lip, orthogonal to the direction of radial migration and ultimately reside in the brainstem. Relationships: is a type of hindbrain tangential cell migration [GO:0021934]